{
  "term_id": "GO:0007169",
  "gene": "UniProtKB:P42685",
  "gene_symbol": "FRK",
  "gene_name": "Tyrosine-protein kinase FRK",
  "term_label": "cell surface receptor protein tyrosine kinase signaling pathway"
}